{
  "term_label": "nucleus",
  "term_id": "GO:0005634",
  "gene_symbol": "CHCHD2P9",
  "gene": "UniProtKB:Q5T1J5",
  "gene_name": "Putative coiled-coil-helix-coiled-coil-helix domain-containing protein CHCHD2P9, mitochondrial"
}